{
  "gene_name": "Volume-regulated anion channel subunit LRRC8D",
  "term_id": "GO:0098656",
  "gene_symbol": "LRRC8D",
  "gene": "UniProtKB:Q7L1W4",
  "term_label": "monoatomic anion transmembrane transport"
}